{
  "gene_symbol": "TIMMDC1",
  "term_id": "GO:0005739",
  "gene_name": "Complex I assembly factor TIMMDC1, mitochondrial",
  "gene": "UniProtKB:Q9NPL8",
  "term_label": "mitochondrion"
}